{
  "gene_name": "Kelch-like protein 26",
  "term_id": "GO:0043161",
  "gene_symbol": "KLHL26",
  "term_label": "proteasome-mediated ubiquitin-dependent protein catabolic process",
  "gene": "UniProtKB:Q53HC5"
}